positive regulation of smooth muscle tissue development [GO:1905901] (BP) Definition: Any process that activates or increases the frequency, rate or extent of smooth muscle tissue development. Also known as: up regulation of smooth muscle tissue development, up-regulation of smooth muscle tissue development, upregulation of smooth muscle tissue development, activation of smooth muscle tissue development References: PMID:14709716 Sources: GOC:TermGenie, GOC:bhm, GO_REF:0000058 Relationships: is a type of positive regulation of muscle tissue development [GO:1901863]; is a type of regulation of smooth muscle tissue development [GO:1905899]; positively regulates GO:0048745